{
  "gene": "UniProtKB:O14926",
  "term_label": "actin filament binding",
  "gene_symbol": "FSCN2",
  "term_id": "GO:0051015",
  "gene_name": "Fascin-2"
}